{
  "term_label": "Unknown cellular component",
  "gene": "UniProtKB:Q8N7Y1",
  "term_id": "UNKNOWN:0003",
  "gene_symbol": "KIRREL3-AS3",
  "gene_name": "Putative uncharacterized protein KIRREL3-AS3"
}